{
  "gene": "UniProtKB:A6NC51",
  "gene_name": "Modulator of macroautophagy TMEM150B",
  "term_id": "UNKNOWN:0001",
  "gene_symbol": "TMEM150B",
  "term_label": "Unknown molecular function"
}